{
  "term_label": "Unknown molecular function",
  "gene_name": "Synapsin-1",
  "gene_symbol": "SYN1",
  "gene": "UniProtKB:P17600",
  "term_id": "UNKNOWN:0001"
}